{
  "gene": "UniProtKB:Q7RTU3",
  "gene_name": "Oligodendrocyte transcription factor 3",
  "term_label": "sensory organ development",
  "term_id": "GO:0007423",
  "gene_symbol": "OLIG3"
}